{
  "gene": "UniProtKB:B2RXH2",
  "gene_symbol": "KDM4E",
  "term_id": "GO:0005634",
  "term_label": "nucleus",
  "gene_name": "Lysine-specific demethylase 4E"
}